regulation of long-chain fatty acid import into cell [GO:0140212] (biological process) Definition: Any process that modulates the frequency, rate or extent of long-chain fatty acid import into a cell. Relationships: is a type of regulation of fatty acid transport [GO:2000191]; regulates long-chain fatty acid import into cell [GO:0044539] Subtypes: regulation of long-chain fatty acid import across plasma membrane [GO:0010746], negative regulation of long-chain fatty acid import into cell [GO:0140213], positive regulation of long-chain fatty acid import into cell [GO:0140214] References: PMID:28178239